{
  "term_id": "GO:0071014",
  "gene_symbol": "CCDC12",
  "term_label": "post-mRNA release spliceosomal complex",
  "gene": "UniProtKB:Q8WUD4",
  "gene_name": "Coiled-coil domain-containing protein 12"
}